{
  "gene": "UniProtKB:Q96GA3",
  "term_id": "GO:0000056",
  "term_label": "ribosomal small subunit export from nucleus",
  "gene_name": "Protein LTV1 homolog",
  "gene_symbol": "LTV1"
}